{
  "term_label": "histone deacetylase complex",
  "gene": "UniProtKB:Q9BY41",
  "gene_name": "Histone deacetylase 8",
  "gene_symbol": "HDAC8",
  "term_id": "GO:0000118"
}